{
  "gene_name": "Ubiquitin-like modifier-activating enzyme 6",
  "gene_symbol": "UBA6",
  "term_label": "cytoplasm",
  "gene": "UniProtKB:A0AVT1",
  "term_id": "GO:0005737"
}